{
  "gene": "UniProtKB:Q86SG7",
  "gene_name": "Lysozyme g-like protein 2",
  "term_id": "GO:0050830",
  "term_label": "defense response to Gram-positive bacterium",
  "gene_symbol": "LYG2"
}